{
  "gene_name": "DNA-directed RNA polymerase I subunit RPA12",
  "gene_symbol": "POLR1H",
  "gene": "UniProtKB:Q9P1U0",
  "term_id": "GO:0006363",
  "term_label": "termination of RNA polymerase I transcription"
}